{
  "gene_symbol": "CCL25",
  "gene": "UniProtKB:O15444",
  "gene_name": "C-C motif chemokine 25",
  "term_id": "GO:0005615",
  "term_label": "extracellular space"
}